{
  "term_label": "nucleus",
  "gene_name": "MyoD family inhibitor",
  "term_id": "GO:0005634",
  "gene": "UniProtKB:Q99750",
  "gene_symbol": "MDFI"
}